{
  "term_id": "UNKNOWN:0003",
  "gene_name": "Sarcoplasmic reticulum histidine-rich calcium-binding protein",
  "gene_symbol": "HRC",
  "term_label": "Unknown cellular component",
  "gene": "UniProtKB:P23327"
}